integrin alphav-beta3 complex [GO:0034683] (cellular component) Definition: An integrin complex that comprises one alphav subunit and one beta3 subunit. References: PMID:12297042 Also known as: alphav-beta3 integrin complex, ITGAV-ITGB3 complex Relationships: is a type of integrin complex [GO:0008305]